{
  "gene_symbol": "MFSD2A",
  "gene": "UniProtKB:Q8NA29",
  "term_id": "GO:0015908",
  "term_label": "fatty acid transport",
  "gene_name": "Sodium-dependent lysophosphatidylcholine symporter 1"
}